intermediate filament bundle assembly [GO:0045110] (biological process) Subtypes: neurofilament bundle assembly [GO:0033693] Sources: ISBN:0716731363 Definition: The formation of the bundles of intermediate filaments. Intermediate filament-associated proteins (IFAPs) cross-link intermediate filaments with one another, forming a bundle or a network, and with other cell structures, including the plasma membrane. The organization of intermediate filaments and their supportive function in various cells types depends in large part on their linkage to other cell structures via IFAPs. Relationships: is a type of cellular component assembly [GO:0022607]; is a type of GO:0045109 Also known as: tonofilament assembly